{
  "term_id": "UNKNOWN:0001",
  "term_label": "Unknown molecular function",
  "gene_symbol": "TRBC2",
  "gene_name": "T cell receptor beta constant 2",
  "gene": "UniProtKB:A0A5B9"
}